inward rectifier potassium channel activity [GO:0005242] (molecular function) Regulation: negatively regulated by inward rectifier potassium channel inhibitor activity [GO:0070320]; negatively regulated by GO:1903609 Also known as: Kir channel activity Relationships: is a type of voltage-gated potassium channel activity [GO:0005249]; is a type of ligand-gated monoatomic cation channel activity [GO:0099094] References: PMID:14977398 Sources: GOC:cb, GOC:mah Subtypes: ATP-activated inward rectifier potassium channel activity [GO:0015272], G-protein activated inward rectifier potassium channel activity [GO:0015467] Definition: Enables the transmembrane transfer of a potassium ion by an inwardly-rectifying voltage-gated channel. An inwardly rectifying current-voltage relation is one where at any given driving force the inward flow of K+ ions exceeds the outward flow for the opposite driving force. The inward-rectification is due to a voltage-dependent block of the channel pore by a specific ligand or ligands, and as a result the macroscopic conductance depends on the difference between membrane voltage and the K+ equilibrium potential rather than on membrane voltage itself.